trans-acenaphthene-1,2-diol dehydrogenase activity [GO:0047062] (molecular function) Sources: EC:1.10.1.1, RHEA:22184 Also known as: (+-)-trans-acenaphthene-1,2-diol:NADP+ oxidoreductase activity, trans-1,2-acenaphthenediol dehydrogenase activity Definition: Catalysis of the reaction: (+-)-trans-acenaphthene-1,2-diol + 2 NADP+ = acenaphthene-1,2-dione + 2 H+ + 2 NADPH. Relationships: is a type of oxidoreductase activity, acting on diphenols and related substances as donors, NAD or NADP as acceptor [GO:0016680]